UDP-N-acetylglucosamine 4-epimerase activity [GO:0003974] (molecular function) Also known as: UDP acetylglucosamine epimerase activity, UDP-GlcNAc 4-epimerase activity, UDP-N-acetyl-D-glucosamine 4-epimerase activity, uridine 5'-diphospho-N-acetylglucosamine-4-epimerase activity, uridine diphosphate N-acetylglucosamine-4-epimerase activity, uridine diphosphoacetylglucosamine epimerase activity Sources: EC:5.1.3.7 Note: Note that this term has a MetaCyc pathway reference as the pathway only has a single step. Relationships: is a type of racemase and epimerase activity, acting on carbohydrates and derivatives [GO:0016857] Definition: Catalysis of the reaction: UDP-N-acetyl-D-glucosamine = UDP-N-acetyl-D-galactosamine.